{
  "term_label": "cytosol",
  "gene": "UniProtKB:O15540",
  "gene_symbol": "FABP7",
  "term_id": "GO:0005829",
  "gene_name": "Fatty acid-binding protein, brain"
}